{
  "term_label": "mitochondrial ATP synthesis coupled electron transport",
  "gene": "UniProtKB:P56181",
  "term_id": "GO:0042775",
  "gene_symbol": "NDUFV3",
  "gene_name": "NADH dehydrogenase [ubiquinone] flavoprotein 3, mitochondrial"
}